{
  "gene_symbol": "DNAH7",
  "term_id": "GO:0051959",
  "gene": "UniProtKB:Q8WXX0",
  "gene_name": "Dynein axonemal heavy chain 7",
  "term_label": "dynein light intermediate chain binding"
}